glial cell-derived neurotrophic factor receptor activity [GO:0016167] (MF) Also known as: GDNF receptor activity, glial cell line-derived neurotrophic factor receptor activity Relationships: is a type of cytokine receptor activity [GO:0004896]; is part of glial cell-derived neurotrophic factor receptor signaling pathway [GO:0035860] Definition: Combining with glial cell line-derived neurotrophic factor and transmitting the signal from one side of the membrane to the other to initiate a change in cell activity. Sources: GOC:mah, GOC:signaling